{
  "term_label": "condensin complex",
  "gene_name": "Condensin complex subunit 1",
  "gene": "UniProtKB:Q15021",
  "term_id": "GO:0000796",
  "gene_symbol": "NCAPD2"
}